{
  "gene": "UniProtKB:Q7Z6M1",
  "term_label": "Unknown cellular component",
  "term_id": "UNKNOWN:0003",
  "gene_name": "Rab9 effector protein with kelch motifs",
  "gene_symbol": "RABEPK"
}